prostaglandin D2 11-ketoreductase activity [GO:0036131] (molecular function) Also known as: PGD2 11-ketoreductase, prostaglandin 11-keto reductase Definition: Catalysis of the reaction: prostaglandin D2 + H+ + NADPH = 11-epi-prostaglandin F2alpha + NADP+. References: PMID:1504718, PMID:3862115 Sources: RHEA:45316 Relationships: is a type of oxidoreductase activity, acting on the CH-OH group of donors, NAD or NADP as acceptor [GO:0016616]; is part of prostaglandin metabolic process [GO:0006693]